{
  "term_label": "calcium ion binding",
  "gene_name": "Protein S100-A7A",
  "gene_symbol": "S100A7A",
  "gene": "UniProtKB:Q86SG5",
  "term_id": "GO:0005509"
}